endosome [GO:0005768] (cellular component) References: PMID:19696797 Sources: ISBN:0198506732 Subtypes: GO:0005769, late endosome [GO:0005770], endolysosome [GO:0036019], GO:0044352, GO:0055037, GO:0097443, presynaptic endosome [GO:0098830], GO:0098845 Definition: A vacuole to which materials ingested by endocytosis are delivered. Relationships: is a type of cytoplasmic vesicle [GO:0031410]; is part of endomembrane system [GO:0012505]